{
  "term_id": "UNKNOWN:0002",
  "gene_name": "Inter-alpha-trypsin inhibitor heavy chain H1",
  "term_label": "Unknown biological process",
  "gene": "UniProtKB:P19827",
  "gene_symbol": "ITIH1"
}